{
  "term_id": "GO:0000278",
  "gene_symbol": "CLTC",
  "gene": "UniProtKB:Q00610",
  "gene_name": "Clathrin heavy chain 1",
  "term_label": "mitotic cell cycle"
}